keto-deoxynonulosonic acid (KDN) cytidylyltransferase activity [GO:0090633] (molecular function) Definition: Catalysis of the reaction: CTP + KDN = diphosphate + CMP-KDN. Also known as: CMP-KDN synthetase activity, cytidine 5'-monophospho-2-Keto-3-deoxy-D-glycero-D-galacto-nononic acid synthetase activity Relationships: is_a cytidylyltransferase activity [GO:0070567] References: PMID:11479279, PMID:8381411 Sources: ISBN:978-1-60805-067-3